{
  "gene_symbol": "ARHGAP22",
  "gene": "UniProtKB:Q7Z5H3",
  "gene_name": "Rho GTPase-activating protein 22",
  "term_label": "Unknown cellular component",
  "term_id": "UNKNOWN:0003"
}